initial mitotic spindle pole body separation [GO:0000073] (biological process) Definition: The release of duplicated mitotic spindle pole bodies (SPBs) that begins with the nucleation of microtubules from each SPB within the nucleus, leading to V-shaped spindle microtubules. Interpolar microtubules that elongate from each pole are interconnected, forming overlapping microtubules. Capturing and antiparallel sliding apart of microtubules promotes the initial separation of the SPB. Relationships: is a type of spindle pole body separation [GO:0110100]; is a type of mitotic cell cycle process [GO:1903047]; is part of mitotic spindle formation (spindle phase one) [GO:0061804]; is part of mitotic spindle pole body organization [GO:1905047] Sources: GOC:sgd_curators, GOC:vw Regulation: regulated by regulation of mitotic spindle pole body separation [GO:0010695]; RO_0002213 by positive regulation of mitotic spindle pole body separation [GO:0010696]; negatively regulated by negative regulation of mitotic spindle pole body separation [GO:0010697]